negative regulation of basidium development [GO:0075316] (biological process) Relationships: is_a GO:0075262; is a type of regulation of basidium development [GO:0075314]; negatively regulates basidium development [GO:0075313] Definition: Any process that stops, prevents, or reduces the frequency, rate or extent of basidium development, a process that leads to the formation of basidium, a small, specialized club-shaped structure typically bearing four basidiospores at the tips of minute projections. The basidium is unique to basidiomycetes and distinguishes them from other kinds of fungi. Sources: GOC:pamgo_curators